{
  "term_label": "autocrine signaling",
  "gene_name": "Protein S100-A9",
  "gene_symbol": "S100A9",
  "term_id": "GO:0035425",
  "gene": "UniProtKB:P06702"
}